biliverdin reductase (NADPH) activity [GO:0106277] (molecular function) Sources: RHEA:15793 Relationships: is a type of biliverdin reductase [NAD(P)H] activity [GO:0004074] Also known as: biliverdin reductase (NADP+) activity Definition: Catalysis of the reaction: bilirubin IXalpha + NADP+ = biliverdin IXalpha + NADPH + H+.